thiocyanate metabolic process [GO:0018969] (biological process) Also known as: thiocyanate metabolism, thiocyanic acid metabolic process, thiocyanic acid metabolism Definition: The chemical reactions and pathways involving thiocyanate, the anion of thiocyanic acid, a toxic cyanide derivative commonly formed as a by-product in the production of gas for fuel, coke, and substances for chemical industries. Relationships: is a type of organic acid metabolic process [GO:0006082]; is a type of sulfur compound metabolic process [GO:0006790]; is a type of xenobiotic metabolic process [GO:0006805] Sources: GOC:jl Subtypes: GO:0046265